{
  "term_id": "UNKNOWN:0002",
  "term_label": "Unknown biological process",
  "gene": "UniProtKB:A0A3B3IS91",
  "gene_name": "POLG alternative reading frame",
  "gene_symbol": "POLGARF"
}